tRNA (guanine(10)-N2)-methyltransferase activity [GO:0160102] (molecular function) Also known as: tRNA (guanine(10)-N(2))-methyltransferase activity, tRNA (guanosine(10)-N(2))-methyltransferase activity Definition: Catalysis of the reaction: guanosine(10) in tRNA + S-adenosyl-L-methionine = H+ + N(2)-methylguanosine(10) in tRNA + S-adenosyl-L-homocysteine. Sources: EC:2.1.1.214 Relationships: is a type of N-methyltransferase activity [GO:0008170]; is a type of GO:0016423